{
  "gene_symbol": "EFCAB8",
  "gene_name": "EF-hand calcium-binding domain-containing protein 8",
  "gene": "UniProtKB:A8MWE9",
  "term_label": "Unknown molecular function",
  "term_id": "UNKNOWN:0001"
}